tRNA acetylation [GO:0051391] (BP) Relationships: is a type of tRNA modification [GO:0006400]; is a type of RNA acetylation [GO:1990884] Definition: The modification of tRNA structure by addition of an acetyl group to tRNA. An acetyl group is CH3CO-, derived from acetic [ethanoic] acid. Sources: GOC:ai